collagen type XXV trimer [GO:1990327] (cellular component) Relationships: is a type of transmembrane collagen trimer [GO:0030936] References: PMID:17876790 Definition: A collagen homotrimer of alpha1(XXV) chains; type XXV collagen triple helices span the plasma membrane.